regulation of methane biosynthetic process from formic acid [GO:1900339] (biological process) Subtypes: GO:1900340, GO:1900341 Definition: Any process that modulates the frequency, rate or extent of methane biosynthetic process from formic acid. Relationships: is a type of regulation of ketone metabolic process [GO:0010565]; is_a regulation of cellular respiration [GO:0043457]; is a type of GO:0062012; is a type of GO:1901577; regulates methane biosynthetic process from formic acid [GO:2001127] Sources: GOC:TermGenie, GOC:mengo_curators